dolichol-phosphate-mannose synthase complex [GO:0033185] (cellular component) References: PMID:10835346 Also known as: DPM synthase complex, dolichyl-phosphate beta-D-mannosyltransferase complex Definition: A protein complex that possesses dolichyl-phosphate beta-D-mannosyltransferase activity; contains a catalytic subunit, a regulatory subunit, and a third subunit that stabilizes the complex. In human and several other metazoa, the subunits are named DPM1, DPM2 and DPM3, respectively. Relationships: is a type of mannosyltransferase complex [GO:0031501]